positive regulation of neutrophil extravasation [GO:2000391] (biological process) Definition: Any process that activates or increases the frequency, rate or extent of neutrophil extravasation. Sources: GOC:BHF, GOC:mah Relationships: is a type of positive regulation of cellular extravasation [GO:0002693]; is a type of positive regulation of neutrophil migration [GO:1902624]; is a type of regulation of neutrophil extravasation [GO:2000389]; positively regulates neutrophil extravasation [GO:0072672]